{
  "term_label": "Unknown cellular component",
  "term_id": "UNKNOWN:0003",
  "gene_name": "Paraneoplastic antigen-like protein 8B",
  "gene_symbol": "PNMA8B",
  "gene": "UniProtKB:Q9ULN7"
}